{
  "gene_name": "Golgi-associated PDZ and coiled-coil motif-containing protein",
  "gene": "UniProtKB:Q9HD26",
  "gene_symbol": "GOPC",
  "term_label": "Golgi apparatus",
  "term_id": "GO:0005794"
}